{
  "gene_name": "Protocadherin gamma-C5",
  "term_label": "plasma membrane",
  "term_id": "GO:0005886",
  "gene_symbol": "PCDHGC5",
  "gene": "UniProtKB:Q9Y5F6"
}